{
  "term_id": "GO:0060070",
  "gene_name": "Protein Wnt-8a",
  "gene_symbol": "WNT8A",
  "term_label": "canonical Wnt signaling pathway",
  "gene": "UniProtKB:Q9H1J5"
}